negative regulation of gluconeogenesis [GO:0045721] (biological process) Definition: Any process that stops, prevents, or reduces the frequency, rate or extent of gluconeogenesis. Sources: GOC:go_curators Also known as: down regulation of gluconeogenesis, down-regulation of gluconeogenesis, downregulation of gluconeogenesis, inhibition of gluconeogenesis Relationships: is a type of GO:0006111; is_a negative regulation of biosynthetic process [GO:0009890]; is a type of negative regulation of carbohydrate metabolic process [GO:0045912]; is a type of negative regulation of small molecule metabolic process [GO:0062014]; negatively regulates gluconeogenesis [GO:0006094]